{
  "term_id": "UNKNOWN:0001",
  "gene_symbol": "LGSN",
  "term_label": "Unknown molecular function",
  "gene_name": "Lengsin",
  "gene": "UniProtKB:Q5TDP6"
}